regulation of seed germination [GO:0010029] (biological process) Definition: Any process that modulates the frequency, rate or extent of seed germination. Sources: GOC:sm Subtypes: positive regulation of seed germination [GO:0010030], negative regulation of seed germination [GO:0010187] Relationships: is a type of regulation of seedling development [GO:1900140]; regulates seed germination [GO:0009845]